{
  "gene_symbol": "COPS8",
  "term_label": "Unknown molecular function",
  "gene_name": "COP9 signalosome complex subunit 8",
  "term_id": "UNKNOWN:0001",
  "gene": "UniProtKB:Q99627"
}